{
  "term_id": "GO:0050911",
  "gene_symbol": "OR2V2",
  "term_label": "detection of chemical stimulus involved in sensory perception of smell",
  "gene_name": "Olfactory receptor 2V2",
  "gene": "UniProtKB:Q96R30"
}